N-acetylgalactosaminyl-proteoglycan 3-beta-glucuronosyltransferase activity [GO:0050510] (molecular function) Definition: Catalysis of the reaction: N-acetyl-beta-D-galactosaminyl-(1,4)-beta-D-glucuronosyl-proteoglycan + UDP-alpha-D-glucuronate = beta-D-glucuronosyl-(1,3)-N-acetyl-beta-D-galactosaminyl-(1,4)-beta-D-glucuronosyl-proteoglycan + UDP. Sources: EC:2.4.1.226 Also known as: N-acetylgalactosaminyl-proteoglycan 3-b-glucuronosyltransferase activity, alpha-D-glucuronate:N-acetyl-beta-D-galactosaminyl-(1->4)-beta-D-glucuronosyl-proteoglycan 3-beta-glucuronosyltransferase activity, chondroitin glucuronyltransferase II activity Relationships: is a type of glucuronosyltransferase activity [GO:0015020]